cephamycin C biosynthetic process [GO:1901118] (biological process) Definition: The chemical reactions and pathways resulting in the formation of cephamycin C. Sources: GOC:TermGenie, GOC:yaf, UniPathway:UPA00183 Also known as: cephamycin C anabolism, cephamycin C biosynthesis, cephamycin C formation, cephamycin C synthesis Relationships: is a type of beta-lactam antibiotic biosynthetic process [GO:0030654]; is a type of sulfur compound biosynthetic process [GO:0044272]